ecdysiostatic hormone activity [GO:0016087] (molecular function) Relationships: is_a GO:0005184 Definition: The action characteristic of ecdysiostatic hormone, a peptide hormone that inhibits ecdysone secretion. Sources: DOI:10.1002/(SICI)1520-6327(1997)35:1, GOC:mah